{
  "gene": "UniProtKB:O14607",
  "term_id": "GO:0010468",
  "gene_symbol": "UTY",
  "term_label": "regulation of gene expression",
  "gene_name": "Histone demethylase UTY"
}